halogenase activity [GO:0140906] (molecular function) Subtypes: haloperoxidase activity [GO:0140905], flavin-dependent halogenase activity [GO:0140907] Definition: Catalysis of the reaction: R-CH + a halogen + oxygen donor = R-C-halogen +H2O. References: PMID:28466644, PMID:34368824 Relationships: is a type of GO:0016705